maintenance of pigment granule location [GO:0051906] (biological process) Sources: GOC:ai, GOC:dph, GOC:tb Definition: Any process in which a pigment granule is maintained in a location and prevented from moving elsewhere. Also known as: maintenance of pigment granule localization Relationships: is a type of GO:0051655; is part of pigment granule localization [GO:0051875]